{
  "term_id": "GO:0006357",
  "gene_name": "Transcription factor Sp4",
  "term_label": "regulation of transcription by RNA polymerase II",
  "gene": "UniProtKB:Q02446",
  "gene_symbol": "SP4"
}